{
  "gene_symbol": "RELT",
  "gene": "UniProtKB:Q969Z4",
  "gene_name": "Tumor necrosis factor receptor superfamily member 19L",
  "term_id": "GO:0097186",
  "term_label": "amelogenesis"
}